{
  "term_label": "SCF ubiquitin ligase complex",
  "gene": "UniProtKB:Q9UJT9",
  "gene_name": "F-box_LRR-repeat protein 7",
  "term_id": "GO:0019005",
  "gene_symbol": "FBXL7"
}